L-lysine alpha-aminotransferase [GO:0062045] (molecular function) References: PMID:27758894, PMID:28330936 Relationships: is a type of transaminase activity [GO:0008483] Definition: Catalysis of the reaction: L-lysine + pyruvate= epsilon-amino-alpha-ketocaproic acid (KAC) + alanine.